response to temozolomide [GO:1990054] (biological process) Sources: GOC:hp Note: Note that this term is in the subset of terms that should not be used for direct manual annotation of gene products. It was created to be used for cross-referencing by other ontologies. Direct annotations to this term may be amended during annotation QC. Definition: Any process that results in a change in state or activity of a cell or an organism (in terms of movement, secretion, enzyme production, gene expression, etc.) as a result of a temozolomide stimulus. Relationships: is a type of response to nitrogen compound [GO:1901698]; is a type of GO:1901700